{
  "gene_symbol": "SLC22A17",
  "gene_name": "Solute carrier family 22 member 17",
  "gene": "UniProtKB:Q8WUG5",
  "term_id": "UNKNOWN:0001",
  "term_label": "Unknown molecular function"
}